regulation of vasoconstriction by norepinephrine [GO:0003116] (biological process) Subtypes: regulation of vasoconstriction by circulating norepinephrine [GO:0003117], regulation of vasoconstriction by neuronal norepinephrine [GO:0003118] Relationships: is a type of regulation of vasoconstriction [GO:0019229] Definition: Any process that modulates the frequency, rate or extent of reductions in the diameter of blood vessels as a result of secretion of norepinephrine into the bloodstream or released by nerve endings. Sources: GOC:mtg_cardio